{
  "gene_name": "Signal peptide, CUB and EGF-like domain-containing protein 1",
  "term_id": "GO:0007165",
  "gene_symbol": "SCUBE1",
  "term_label": "signal transduction",
  "gene": "UniProtKB:Q8IWY4"
}